{
  "term_id": "GO:0051607",
  "gene": "UniProtKB:Q96AZ6",
  "gene_symbol": "ISG20",
  "term_label": "defense response to virus",
  "gene_name": "Interferon-stimulated gene 20 kDa protein"
}